response to menaquinone [GO:0032572] (biological process) Also known as: response to menatetrenone, response to vitamin K2 Relationships: is a type of response to vitamin K [GO:0032571] Definition: Any process that results in a change in state or activity of a cell or an organism (in terms of movement, secretion, enzyme production, gene expression, etc.) as a result of a menaquinone (vitamin K2) stimulus. Sources: GOC:sl Subtypes: cellular response to menaquinone [GO:0071308]